dephosphorylation [GO:0016311] (biological process) Sources: ISBN:0198506732 Subtypes: protein dephosphorylation [GO:0006470], GO:0035644, GO:0046839, GO:0098506, GO:0098507 Relationships: is a type of phosphate-containing compound metabolic process [GO:0006796] Definition: The process of removing one or more phosphoric (ester or anhydride) residues from a molecule. Regulation: regulated by regulation of dephosphorylation [GO:0035303]; negatively regulated by negative regulation of dephosphorylation [GO:0035305]; positively regulated by GO:0035306